{
  "gene": "UniProtKB:P06865",
  "gene_symbol": "HEXA",
  "term_label": "glycosaminoglycan metabolic process",
  "term_id": "GO:0030203",
  "gene_name": "Beta-hexosaminidase subunit alpha"
}